{
  "term_id": "GO:0004465",
  "gene": "UniProtKB:Q9Y4D2",
  "term_label": "lipoprotein lipase activity",
  "gene_symbol": "DAGLA",
  "gene_name": "Diacylglycerol lipase-alpha"
}